{
  "term_id": "UNKNOWN:0001",
  "gene": "UniProtKB:Q9UI54",
  "gene_name": "Putative uncharacterized protein PRO0628",
  "term_label": "Unknown molecular function",
  "gene_symbol": "PRO0628"
}